{
  "gene_symbol": "GHITM",
  "term_id": "GO:0005743",
  "gene": "UniProtKB:Q9H3K2",
  "term_label": "mitochondrial inner membrane",
  "gene_name": "Growth hormone-inducible transmembrane protein"
}